{
  "term_id": "GO:0005549",
  "gene": "UniProtKB:Q8NG78",
  "term_label": "odorant binding",
  "gene_symbol": "OR8G5",
  "gene_name": "Olfactory receptor 8G5"
}